regulation of cell communication [GO:0010646] (biological process) Definition: Any process that modulates the frequency, rate or extent of cell communication. Cell communication is the process that mediates interactions between a cell and its surroundings. Encompasses interactions such as signaling or attachment between one cell and another cell, between a cell and an extracellular matrix, or between a cell and any other aspect of its environment. Sources: GOC:dph, GOC:tb Subtypes: regulation of cell communication involved in growth plate cartilage morphogenesis [GO:0003437], regulation of signal transduction [GO:0009966], GO:0010645, positive regulation of cell communication [GO:0010647], negative regulation of cell communication [GO:0010648], regulation of cell communication by electrical coupling [GO:0010649], regulation of hormone secretion [GO:0046883], regulation of transmission of nerve impulse [GO:0051969], regulation of Wnt protein secretion [GO:0061356], regulation of c-di-GMP signaling [GO:0061940], regulation of AV node cell action potential [GO:0098904], regulation of Purkinje myocyte action potential [GO:0098906], regulation of SA node cell action potential [GO:0098907], GO:0099177, regulation of synaptic signaling by nitric oxide [GO:0150045], regulation of trichome patterning [GO:1900032], regulation of BMP secretion [GO:2001284] Relationships: is a type of GO:0050794; regulates cell communication [GO:0007154]